{
  "gene_name": "Piwi-like protein 4",
  "gene": "UniProtKB:Q7Z3Z4",
  "term_id": "GO:0005634",
  "gene_symbol": "PIWIL4",
  "term_label": "nucleus"
}